{
  "gene_symbol": "SEC11B",
  "gene_name": "Putative signal peptidase complex catalytic subunit SEC11B",
  "term_label": "signal peptide processing",
  "gene": "UniProtKB:P0C7V7",
  "term_id": "GO:0006465"
}